{
  "term_id": "GO:0015630",
  "gene": "UniProtKB:O75602",
  "term_label": "microtubule cytoskeleton",
  "gene_symbol": "SPAG6",
  "gene_name": "Sperm-associated antigen 6"
}